{
  "gene": "UniProtKB:P31629",
  "gene_symbol": "HIVEP2",
  "term_id": "GO:0000981",
  "gene_name": "Transcription factor HIVEP2",
  "term_label": "DNA-binding transcription factor activity, RNA polymerase II-specific"
}